insulin receptor signaling pathway [GO:0008286] (biological process) Relationships: is a type of GO:0007169; is part of cellular response to insulin stimulus [GO:0032869] Regulation: regulated by regulation of insulin receptor signaling pathway [GO:0046626]; negatively regulated by negative regulation of insulin receptor signaling pathway [GO:0046627]; positively regulated by positive regulation of insulin receptor signaling pathway [GO:0046628] Sources: GOC:ceb Also known as: insulin receptor signalling pathway, daf-2 receptor signaling pathway Definition: The series of molecular signals generated as a consequence of the insulin receptor binding to insulin.